post-anaphase microtubule array [GO:1990295] (cellular component) References: PMID:11792817, PMID:17072892, PMID:9601091 Definition: A cytoskeletal part that consists of an array of microtubules and associated molecules that forms at the end of anaphase, and in which microtubules are nucleated from an equatorial microtubule organizing center. Also known as: PAA, post-anaphase array Relationships: is a type of cellular anatomical structure [GO:0110165]; is part of microtubule cytoskeleton [GO:0015630]; has part equatorial microtubule organizing center [GO:0000923] Note: The best-characterized example is found in the fission yeast Schizosaccharomyces pombe. The eMTOC is cortical, but the post-anaphase array microtubules are not exclusively cortical.